{
  "term_label": "nucleus",
  "term_id": "GO:0005634",
  "gene": "UniProtKB:P52701",
  "gene_symbol": "MSH6",
  "gene_name": "DNA mismatch repair protein Msh6"
}